{
  "gene": "UniProtKB:P51513",
  "term_label": "mRNA splicing, via spliceosome",
  "gene_symbol": "NOVA1",
  "gene_name": "RNA-binding protein Nova-1",
  "term_id": "GO:0000398"
}